{
  "gene_name": "Major vault protein",
  "gene": "UniProtKB:Q14764",
  "term_label": "Unknown biological process",
  "gene_symbol": "MVP",
  "term_id": "UNKNOWN:0002"
}